ribosomal large subunit assembly [GO:0000027] (biological process) References: PMID:30467428 Sources: GOC:jl Also known as: 50S ribosomal subunit assembly, 60S ribosomal subunit assembly Relationships: is a type of protein-RNA complex assembly [GO:0022618]; is part of GO:0042255; is part of ribosomal large subunit biogenesis [GO:0042273] Definition: The aggregation, arrangement and bonding together of constituent RNAs and proteins to form the large ribosomal subunit. Subtypes: cytosolic large ribosomal subunit assembly [GO:0180023], mitochondrial large ribosomal subunit assembly [GO:1902775]